regulation of piRNA transcription [GO:0140542] (biological process) Subtypes: positive regulation of piRNA transcription [GO:0140543] Relationships: is a type of GO:0006355; regulates GO:0140541 Definition: Any process that modulates the frequency, rate or extent of the synthesis of a piRNA. References: PMID:28847004